{
  "gene_symbol": "ZBTB8A",
  "gene_name": "Zinc finger and BTB domain-containing protein 8A",
  "term_id": "GO:0000981",
  "term_label": "DNA-binding transcription factor activity, RNA polymerase II-specific",
  "gene": "UniProtKB:Q96BR9"
}